{
  "gene_name": "Nanos homolog 2",
  "term_label": "perinuclear region of cytoplasm",
  "gene": "UniProtKB:P60321",
  "gene_symbol": "NANOS2",
  "term_id": "GO:0048471"
}